response to corticosteroid [GO:0031960] (biological process) References: PMID:11027914 Sources: GOC:mah Definition: Any process that results in a change in state or activity of a cell or an organism (in terms of movement, secretion, enzyme production, gene expression, etc.) as a result of a corticosteroid hormone stimulus. A corticosteroid is a steroid hormone that is produced in the adrenal cortex. Corticosteroids are involved in a wide range of physiologic systems such as stress response, immune response and regulation of inflammation, carbohydrate metabolism, protein catabolism, blood electrolyte levels, and behavior. They include glucocorticoids and mineralocorticoids. Relationships: is a type of GO:0048545 Subtypes: response to glucocorticoid [GO:0051384], response to mineralocorticoid [GO:0051385], cellular response to corticosteroid stimulus [GO:0071384] Also known as: response to corticosteroid stimulus